animal organ formation [GO:0048645] (biological process) Also known as: animal organ primordium initiation, initiation of an animal organ primordium Relationships: is a type of GO:0048646; is part of animal organ morphogenesis [GO:0009887] Sources: GOC:dph, GOC:jid Definition: The process pertaining to the initial formation of an animal organ from unspecified parts. The process begins with the specific processes that contribute to the appearance of the discrete structure, such as inductive events, and ends when the structural rudiment of the organ is recognizable, such as a condensation of mesenchymal cells into the organ rudiment. Organs are a natural part or structure in an animal or a plant, capable of performing some special action (termed its function), which is essential to the life or well-being of the whole. The heart and lungs are organs of animals, and the petal and leaf are organs of plants. In animals the organs are generally made up of several tissues, one of which usually predominates, and determines the principal function of the organ. Subtypes: swim bladder formation [GO:0048797], GO:0060431, trachea formation [GO:0060440], prostatic bud formation [GO:0060513], GO:0060914, GO:0061130, GO:0072116 Regulation: regulated by regulation of animal organ formation [GO:0003156]